{
  "term_id": "GO:0047555",
  "gene_name": "High affinity cAMP-specific and IBMX-insensitive 3',5'-cyclic phosphodiesterase 8A",
  "term_label": "3',5'-cyclic-GMP phosphodiesterase activity",
  "gene_symbol": "PDE8A",
  "gene": "UniProtKB:O60658"
}